{
  "term_label": "Unknown molecular function",
  "gene_symbol": "TRAV8-1",
  "gene_name": "T cell receptor alpha variable 8-1",
  "gene": "UniProtKB:A0A0A6YYK1",
  "term_id": "UNKNOWN:0001"
}